growth cone [GO:0030426] (cellular component) Relationships: is a type of GO:0030427; is part of distal axon [GO:0150034] References: PMID:10082468 Sources: GOC:aruk, GOC:bc, ISBN:0815316194 Definition: The migrating motile tip of a growing neuron projection, where actin accumulates, and the actin cytoskeleton is the most dynamic. Subtypes: dendritic growth cone [GO:0044294], axonal growth cone [GO:0044295]